{
  "gene": "UniProtKB:O43237",
  "gene_symbol": "DYNC1LI2",
  "term_label": "microtubule-based movement",
  "term_id": "GO:0007018",
  "gene_name": "Cytoplasmic dynein 1 light intermediate chain 2"
}